{
  "gene_name": "Lupus La protein",
  "term_label": "mRNA binding",
  "term_id": "GO:0003729",
  "gene_symbol": "SSB",
  "gene": "UniProtKB:P05455"
}